protein-N(PI)-phosphohistidine-N-acetylglucosamine phosphotransferase system transporter activity [GO:0022880] (molecular function) Relationships: is a type of protein-N(PI)-phosphohistidine-sugar phosphotransferase activity [GO:0008982]; is_a N-acetylglucosamine transmembrane transporter activity [GO:0015572] Definition: Catalysis of the PEP-dependent, phosphoryl transfer-driven transport of substances across a membrane. The transport happens by catalysis of the reaction: protein N-phosphohistidine + N-acetylglucosamine(out) = protein histidine + N-acetylglucosamine phosphate(in). This differs from primary and secondary active transport in that the solute is modified during transport. Also known as: N-acetylglucosamine PTS transporter activity Sources: GOC:mtg_transport, ISBN:0815340729